{
  "gene": "UniProtKB:Q96D46",
  "gene_symbol": "NMD3",
  "term_label": "ribosomal large subunit binding",
  "term_id": "GO:0043023",
  "gene_name": "60S ribosomal export protein NMD3"
}